{
  "term_label": "Unknown biological process",
  "gene": "UniProtKB:Q8NH54",
  "term_id": "UNKNOWN:0002",
  "gene_symbol": "OR56A3",
  "gene_name": "Olfactory receptor 56A3"
}